{
  "gene_symbol": "SPDYE17",
  "gene_name": "Putative speedy protein E17",
  "term_id": "GO:0019901",
  "term_label": "protein kinase binding",
  "gene": "UniProtKB:P0DUD2"
}